isopullulanase activity [GO:0051675] (molecular function) Sources: EC:3.2.1.57 Also known as: pullulan 4-glucanohydrolase (isopanose-forming) activity Relationships: is_a hydrolase activity, hydrolyzing O-glycosyl compounds [GO:0004553] Definition: Catalysis of the hydrolysis of pullulan to isopanose (6-alpha-maltosylglucose).